aconitate delta-isomerase activity [GO:0047614] (molecular function) Also known as: aconitate isomerase activity, aconitate D-isomerase activity, aconitate delta2-delta3-isomerase activity Sources: RHEA:17265 Definition: Catalysis of the reaction: trans-aconitate = cis-aconitate. Relationships: is a type of intramolecular oxidoreductase activity, transposing C=C bonds [GO:0016863]